{
  "term_id": "GO:0005789",
  "gene_symbol": "TM7SF2",
  "gene_name": "Delta(14)-sterol reductase TM7SF2",
  "term_label": "endoplasmic reticulum membrane",
  "gene": "UniProtKB:O76062"
}